N-acetyltransferase activity [GO:0008080] (MF) Definition: Catalysis of the transfer of an acetyl group to a nitrogen atom on the acceptor molecule. Subtypes: aralkylamine N-acetyltransferase activity [GO:0004059], arylamine N-acetyltransferase activity [GO:0004060], GO:0004145, glucosamine 6-phosphate N-acetyltransferase activity [GO:0004343], heparan-alpha-glucosaminide N-acetyltransferase activity [GO:0015019], glucosamine-1-phosphate N-acetyltransferase activity [GO:0019134], aminoglycoside N-acetyltransferase activity [GO:0034069], protein N-acetyltransferase activity [GO:0034212], alpha-aminoadipate acetyltransferase activity [GO:0043741], azetidine-2-carboxylic acid acetyltransferase activity [GO:0046941], tetrahydrodipicolinate N-acetyltransferase activity [GO:0047200], imidazole N-acetyltransferase activity [GO:0047716], D-amino-acid N-acetyltransferase activity [GO:0047812], glucosamine N-acetyltransferase activity [GO:0047932], tRNA cytidine N4-acetyltransferase activity [GO:0051392], mRNA N-acetyltransferase activity [GO:0106162], L-amino-acid N-acetyltransferase activity [GO:0140085], 18S rRNA cytidine N-acetyltransferase activity [GO:1990883] Sources: GOC:ai Relationships: is a type of acetyltransferase activity [GO:0016407]; is a type of N-acyltransferase activity [GO:0016410]